{
  "gene_symbol": "PHYHIP",
  "term_id": "UNKNOWN:0001",
  "term_label": "Unknown molecular function",
  "gene": "UniProtKB:Q92561",
  "gene_name": "Phytanoyl-CoA hydroxylase-interacting protein"
}